{
  "gene": "UniProtKB:Q9Y5U8",
  "term_label": "pyruvate transmembrane transporter activity",
  "gene_symbol": "MPC1",
  "term_id": "GO:0050833",
  "gene_name": "Mitochondrial pyruvate carrier 1"
}